thiosulfate-dithiol sulfurtransferase activity [GO:0047362] (molecular function) Also known as: thiosulphate-dithiol sulphurtransferase activity, TSR, thiosulfate reductase activity, thiosulfate:dithioerythritol sulfurtransferase activity Relationships: is a type of sulfurtransferase activity [GO:0016783] Definition: Catalysis of the reaction: dithioerythritol + thiosulfate = hydrogen sulfide + dithioerythritol disulfide + sulfite. Sources: EC:2.8.1.5